GW body [GO:0140364] (cellular component) References: PMID:16418578, PMID:26930655, PMID:29576456 Definition: A ribonucleoprotein granule located in the cytoplasm and the nucleus. GW-bodies minimally contain the Argonaute2 (Ago2) and TNRC6B proteins, together with specific target RNAs. Also known as: GW-body Relationships: is a type of cytoplasmic ribonucleoprotein granule [GO:0036464]